{
  "gene_symbol": "FAM149B1",
  "term_id": "GO:0061512",
  "gene_name": "Primary cilium assembly protein FAM149B1",
  "gene": "UniProtKB:Q96BN6",
  "term_label": "protein localization to cilium"
}